{
  "gene_symbol": "LINC00242",
  "gene": "UniProtKB:Q5T6M2",
  "term_label": "Unknown cellular component",
  "gene_name": "Putative uncharacterized protein encoded by LINC00242",
  "term_id": "UNKNOWN:0003"
}